mitochondrial coenzyme A transmembrane transport [GO:1990559] (biological process) References: PMID:11158296 Definition: The process in which coenzyme A is transported across a mitochondrial membrane, into or out of the mitochondrion. Relationships: is a type of GO:0035349